{
  "term_id": "UNKNOWN:0002",
  "gene": "UniProtKB:Q9H3N1",
  "gene_name": "Thioredoxin-related transmembrane protein 1",
  "term_label": "Unknown biological process",
  "gene_symbol": "TMX1"
}